{
  "term_id": "GO:0000150",
  "gene": "UniProtKB:Q14565",
  "term_label": "DNA strand exchange activity",
  "gene_symbol": "DMC1",
  "gene_name": "Meiotic recombination protein DMC1_LIM15 homolog"
}